nucleus localization [GO:0051647] (biological process) Also known as: cell nucleus localization, establishment and maintenance of nucleus localization, localization of nucleus, nucleus localisation Relationships: is a type of GO:0051640 Definition: Any process in which the nucleus is transported to, and/or maintained in, a specific location within the cell. Subtypes: nuclear migration [GO:0007097], nurse cell nucleus anchoring [GO:0007302], maintenance of nucleus location [GO:0051658], oocyte nucleus localization involved in oocyte dorsal/ventral axis specification [GO:0051663] Sources: GOC:ai